{
  "term_label": "Unknown cellular component",
  "gene_name": "Keratin-associated protein 15-1",
  "gene": "UniProtKB:Q3LI76",
  "term_id": "UNKNOWN:0003",
  "gene_symbol": "KRTAP15-1"
}